{
  "gene_name": "Testis-specific Y-encoded protein 9",
  "term_label": "histone binding",
  "term_id": "GO:0042393",
  "gene_symbol": "TSPY9",
  "gene": "UniProtKB:A0A494C1R9"
}